{
  "gene": "UniProtKB:P28328",
  "gene_name": "Peroxisome biogenesis factor 2",
  "gene_symbol": "PEX2",
  "term_label": "fatty acid beta-oxidation",
  "term_id": "GO:0006635"
}